(1->3)-alpha-glucan biosynthetic process [GO:0070596] (biological process) Sources: GOC:mah Subtypes: GO:0070598 Regulation: RO_0002211 by GO:0070606 Definition: The chemical reactions and pathways resulting in the formation of (1->3)-alpha-D-glucans, compounds composed of glucose residues linked by (1->3)-alpha-D-glucosidic bonds. Relationships: is a type of alpha-glucan biosynthetic process [GO:0030979]; is a type of GO:0070595 Also known as: 1,3-alpha-glucan anabolism, 1,3-alpha-glucan biosynthesis, 1,3-alpha-glucan biosynthetic process, 1,3-alpha-glucan formation, 1,3-alpha-glucan synthesis, alpha-1,3 glucan anabolism, alpha-1,3 glucan biosynthesis, alpha-1,3 glucan biosynthetic process, alpha-1,3 glucan formation, alpha-1,3 glucan synthesis